{
  "gene": "UniProtKB:Q9Y2R2",
  "term_label": "nucleus",
  "gene_symbol": "PTPN22",
  "term_id": "GO:0005634",
  "gene_name": "Tyrosine-protein phosphatase non-receptor type 22"
}